{
  "gene_symbol": "FGF7",
  "gene": "UniProtKB:P21781",
  "term_id": "GO:0008543",
  "gene_name": "Fibroblast growth factor 7",
  "term_label": "fibroblast growth factor receptor signaling pathway"
}